{
  "gene_symbol": "UNG",
  "term_label": "base-excision repair, AP site formation via deaminated base removal",
  "term_id": "GO:0097510",
  "gene_name": "Uracil-DNA glycosylase",
  "gene": "UniProtKB:P13051"
}